leucyl-tRNA--protein transferase activity [GO:0008914] (molecular function) Also known as: L/F transferase activity, leucyl-phenylalanine-transfer ribonucleate-protein aminoacyltransferase activity, leucyl-phenylalanine-transfer ribonucleate-protein transferase activity, leucyltransferase activity Sources: EC:2.3.2.6 Relationships: is a type of aminoacyltransferase activity [GO:0016755]; is a type of catalytic activity, acting on a protein [GO:0140096]; is a type of catalytic activity, acting on a tRNA [GO:0140101] Definition: Catalysis of the reaction: L-leucyl-tRNA(Leu) + N-terminal L-arginyl-[protein] = H+ + N-terminal L-leucyl-L-arginyl-[protein] + tRNA(Leu). Can also transfer the leucyl residue on an N-terminal L-lysyl residue.